{
  "gene": "UniProtKB:Q9Y3I0",
  "gene_symbol": "RTCB",
  "term_id": "GO:0170057",
  "term_label": "RNA ligase (GTP) activity",
  "gene_name": "RNA-splicing ligase RtcB homolog"
}